negative regulation of proteasomal protein catabolic process [GO:1901799] (BP) References: PMID:21669198 Sources: GOC:BHF, GOC:TermGenie, GOC:rl Subtypes: GO:0032435, negative regulation of ERAD pathway [GO:1904293] Relationships: is a type of negative regulation of protein catabolic process [GO:0042177]; is_a regulation of proteasomal protein catabolic process [GO:0061136]; is a type of negative regulation of proteolysis involved in protein catabolic process [GO:1903051]; negatively regulates GO:0010498 Definition: Any process that stops, prevents or reduces the frequency, rate or extent of proteasomal protein catabolic process. Also known as: down regulation of proteasomal protein catabolic process, down regulation of proteasome-mediated protein catabolic process, down regulation of proteasome-mediated protein catabolism, down-regulation of proteasomal protein catabolic process, down-regulation of proteasome-mediated protein catabolic process, down-regulation of proteasome-mediated protein catabolism, downregulation of proteasomal protein catabolic process, downregulation of proteasome-mediated protein catabolic process, downregulation of proteasome-mediated protein catabolism, inhibition of proteasome-mediated protein catabolic process, inhibition of proteasome-mediated protein catabolism, negative regulation of proteasome-mediated protein catabolic process, negative regulation of proteasome-mediated protein catabolism, inhibition of proteasomal protein catabolic process